{
  "gene_name": "Beclin-2",
  "term_label": "cellular response to nitrogen starvation",
  "term_id": "GO:0006995",
  "gene_symbol": "BECN2",
  "gene": "UniProtKB:A8MW95"
}